{
  "gene_symbol": "MYRFL",
  "term_id": "GO:0005634",
  "gene": "UniProtKB:Q96LU7",
  "term_label": "nucleus",
  "gene_name": "Myelin regulatory factor-like protein"
}